{
  "term_label": "delayed rectifier potassium channel activity",
  "term_id": "GO:0005251",
  "gene": "UniProtKB:Q96PR1",
  "gene_name": "Potassium voltage-gated channel subfamily C member 2",
  "gene_symbol": "KCNC2"
}